negative regulation of meiotic DNA double-strand break formation involved in reciprocal meiotic recombination [GO:1905262] (biological process) Definition: Any process that stops, prevents or reduces the frequency, rate or extent of meiotic DNA double-strand break formation involved in reciprocal meiotic recombination. References: PMID:26653857 Sources: GOC:TermGenie, GO_REF:0000058 Also known as: down regulation of meiotic DNA double-strand break formation involved in reciprocal meiotic recombination, down-regulation of meiotic DNA double-strand break formation involved in reciprocal meiotic recombination, downregulation of meiotic DNA double-strand break formation involved in reciprocal meiotic recombination, inhibition of meiotic DNA double-strand break formation involved in reciprocal meiotic recombination Relationships: is a type of negative regulation of meiotic DNA double-strand break formation [GO:1903342]; is a type of GO:1905261; negatively regulates meiotic DNA double-strand break formation involved in reciprocal meiotic recombination [GO:0010780]